negative regulation of T cell migration [GO:2000405] (biological process) Definition: Any process that stops, prevents or reduces the frequency, rate or extent of T cell migration. Sources: GOC:mah Also known as: negative regulation of T lymphocyte migration, negative regulation of T-cell migration, negative regulation of T-lymphocyte migration Relationships: is a type of negative regulation of lymphocyte migration [GO:2000402]; is_a regulation of T cell migration [GO:2000404]; negatively regulates T cell migration [GO:0072678] Subtypes: GO:2000408, GO:2000411